iron-sulfur cluster binding [GO:0051536] (molecular function) Relationships: is a type of GO:0051540 Also known as: Fe/S binding, iron sulfur cluster binding, iron sulphur cluster binding, iron-sulphur cluster binding Definition: Binding to an iron-sulfur cluster, a combination of iron and sulfur atoms. Sources: GOC:ai Subtypes: iron-sulfur-molybdenum cofactor binding [GO:0044590], 2 iron, 2 sulfur cluster binding [GO:0051537], 3 iron, 4 sulfur cluster binding [GO:0051538], GO:0051539, 4 iron, 3 sulfur cluster binding [GO:1990655]